{
  "gene": "UniProtKB:P29323",
  "gene_symbol": "EPHB2",
  "gene_name": "Ephrin type-B receptor 2",
  "term_label": "dendrite",
  "term_id": "GO:0030425"
}